{
  "term_id": "UNKNOWN:0002",
  "gene_name": "Sialate:O-sulfotransferase 2",
  "gene": "UniProtKB:Q2TBF2",
  "gene_symbol": "WSCD2",
  "term_label": "Unknown biological process"
}